{
  "gene_symbol": "FBXL8",
  "gene_name": "F-box_LRR-repeat protein 8",
  "term_label": "Unknown molecular function",
  "gene": "UniProtKB:Q96CD0",
  "term_id": "UNKNOWN:0001"
}